{
  "term_label": "RNA polymerase II cis-regulatory region sequence-specific DNA binding",
  "gene_name": "Zinc finger protein Pegasus",
  "term_id": "GO:0000978",
  "gene": "UniProtKB:Q9H5V7",
  "gene_symbol": "IKZF5"
}